positive regulation of fever generation by prostaglandin biosynthetic process [GO:0100010] (BP) Sources: GOC:cjm, GOC:obol Definition: Any prostaglandin biosynthetic process process that positively_regulates fever generation. Relationships: is a type of GO:0100008; positively regulates GO:0001660